{
  "gene_symbol": "ANKRD13C",
  "term_id": "GO:0005102",
  "term_label": "signaling receptor binding",
  "gene": "UniProtKB:Q8N6S4",
  "gene_name": "Ankyrin repeat domain-containing protein 13C"
}